regulation of peptidyl-cysteine S-nitrosylation [GO:2000169] (biological process) Definition: Any process that modulates the frequency, rate or extent of peptidyl-cysteine S-nitrosylation. Sources: GOC:obol Relationships: is_a regulation of protein modification process [GO:0031399]; regulates peptidyl-cysteine S-nitrosylation [GO:0018119] Subtypes: GO:1902083, GO:2000170